{
  "term_label": "T cell activation",
  "gene": "UniProtKB:P10809",
  "gene_name": "60 kDa heat shock protein, mitochondrial",
  "gene_symbol": "HSPD1",
  "term_id": "GO:0042110"
}